{
  "gene": "UniProtKB:P10828",
  "gene_name": "Thyroid hormone receptor beta",
  "gene_symbol": "THRB",
  "term_id": "GO:0048384",
  "term_label": "retinoic acid receptor signaling pathway"
}